{
  "gene": "UniProtKB:Q7Z388",
  "term_label": "mannosyltransferase activity",
  "gene_name": "Probable C-mannosyltransferase DPY19L4",
  "gene_symbol": "DPY19L4",
  "term_id": "GO:0000030"
}